{
  "term_id": "GO:0016493",
  "gene_symbol": "CCR5",
  "gene_name": "C-C chemokine receptor type 5",
  "gene": "UniProtKB:P51681",
  "term_label": "C-C chemokine receptor activity"
}